{
  "gene_name": "Humanin-like 2",
  "term_label": "Unknown cellular component",
  "gene_symbol": "MTRNR2L2",
  "term_id": "UNKNOWN:0003",
  "gene": "UniProtKB:P0CJ69"
}